regulation of cell adhesion involved in heart morphogenesis [GO:0061344] (biological process) Definition: Any process that modulates the extent of cell adhesion contributing to the shaping of the heart. References: PMID:16860783 Sources: GOC:dph, GOC:mtg_heart Relationships: is a type of GO:0030155; regulates cell adhesion involved in heart morphogenesis [GO:0061343]